long-chain fatty acid omega-hydroxylase activity [GO:0102033] (molecular function) Relationships: is a type of GO:0120250 References: PMID:18544608 Sources: GOC:krc, RHEA:56748 Definition: Catalysis of the reaction: an omega-methyl-long-chain fatty acid + O2 + reduced [NADPH--hemoprotein reductase] = an omega-hydroxy-long-chain fatty acid + H+ + H2O + oxidized [NADPH--hemoprotein reductase]. A long-chain fatty acid has an aliphatic tail containing 13 to 22 carbons. Note: While there is not universal consensus on the lengths of short-, medium-, long- and very-long-chain fatty acids, the GO uses the definitions in ChEBI (see CHEBI:26666, CHEBI:59554, CHEBI:15904 and CHEBI:27283). Also known as: cytochrome P450 fatty acid omega-hydroxylase activity